{
  "term_id": "GO:0051455",
  "gene_name": "Centromere protein C",
  "gene": "UniProtKB:Q03188",
  "term_label": "spindle attachment to meiosis I kinetochore",
  "gene_symbol": "CENPC"
}